{
  "gene_symbol": "PGM5",
  "term_label": "Unknown molecular function",
  "term_id": "UNKNOWN:0001",
  "gene_name": "Phosphoglucomutase-like protein 5",
  "gene": "UniProtKB:Q15124"
}